{
  "term_id": "GO:0005737",
  "gene": "UniProtKB:Q15813",
  "term_label": "cytoplasm",
  "gene_symbol": "TBCE",
  "gene_name": "Tubulin-specific chaperone E"
}